{
  "term_id": "UNKNOWN:0001",
  "gene_symbol": "KNSTRN",
  "gene_name": "Small kinetochore-associated protein",
  "gene": "UniProtKB:Q9Y448",
  "term_label": "Unknown molecular function"
}